{
  "gene_name": "Putative uncharacterized protein TSPEAR-AS2",
  "gene": "UniProtKB:P59090",
  "term_label": "Unknown cellular component",
  "term_id": "UNKNOWN:0003",
  "gene_symbol": "TSPEAR-AS2"
}